endonucleolytic cleavage to generate mature 3'-end of SSU-rRNA from (SSU-rRNA, 5.8S rRNA, LSU-rRNA) [GO:0000461] (biological process) Also known as: endonucleolytic cleavage at site D Relationships: is a type of endonucleolytic cleavage of tricistronic rRNA transcript (SSU-rRNA, 5.8S rRNA, LSU-rRNA) [GO:0000479]; is a type of rRNA 3'-end processing [GO:0031125]; BFO_0000050 maturation of SSU-rRNA from tricistronic rRNA transcript (SSU-rRNA, 5.8S rRNA, LSU-rRNA) [GO:0000462] References: PMID:10690410 Sources: GOC:krc Definition: Endonucleolytic cleavage at the 3'-end of the SSU-rRNA from an originally tricistronic rRNA transcript that contained the Small Subunit (SSU) rRNA, the 5.8S rRNA, and the Large Subunit (LSU) rRNA in that order from 5' to 3' along the primary transcript, to produce the mature end of the SSU-rRNA.